L-leucine dehydrogenase activity [GO:0050049] (molecular function) Sources: EC:1.4.1.9 Definition: Catalysis of the reaction: L-leucine + H2O + NAD+ = 4-methyl-2-oxopentanoate + NH3 + NADH. Also known as: L-leucine:NAD+ oxidoreductase (deaminating), L-leucine:NAD+ oxidoreductase, deaminating, LeuDH activity, leucine dehydrogenase activity Relationships: is a type of oxidoreductase activity, acting on the CH-NH2 group of donors, NAD or NADP as acceptor [GO:0016639]